{
  "gene_symbol": "PRCC",
  "gene": "UniProtKB:Q92733",
  "term_label": "Unknown biological process",
  "gene_name": "Proline-rich protein PRCC",
  "term_id": "UNKNOWN:0002"
}